{
  "gene_name": "Microtubule-associated serine_threonine-protein kinase 2",
  "term_id": "GO:0004674",
  "gene": "UniProtKB:Q6P0Q8",
  "term_label": "protein serine/threonine kinase activity",
  "gene_symbol": "MAST2"
}